{
  "term_id": "UNKNOWN:0001",
  "gene": "UniProtKB:Q75V66",
  "gene_symbol": "ANO5",
  "term_label": "Unknown molecular function",
  "gene_name": "Anoctamin-5"
}